{
  "gene_symbol": "S100A14",
  "term_id": "GO:0048306",
  "gene_name": "Protein S100-A14",
  "gene": "UniProtKB:Q9HCY8",
  "term_label": "calcium-dependent protein binding"
}